glucuronoside catabolic process [GO:0019391] (biological process) References: PMID:28389557 Definition: The chemical reactions and pathways resulting in the breakdown of glucuronosides, compound composed of a hydroxy compound linked to a glucuronate residue. Relationships: is a type of GO:0016139 Also known as: glucuronide catabolic process, glucuronide catabolism, glucuronoside breakdown, glucuronoside catabolism, glucuronoside degradation Note: Note that this term was reinstated from obsolete.